protein-folding chaperone binding [GO:0051087] (molecular function) Definition: Binding to a chaperone protein, a class of proteins that bind to nascent or unfolded polypeptides and ensure correct folding or transport. Subtypes: Hsp70 protein binding [GO:0030544] References: PMID:10585443 Relationships: is a type of protein binding [GO:0005515] Also known as: chaperone binding, chaperone protein binding, co-chaperone activity, co-chaperonin activity